{
  "term_id": "GO:0005794",
  "gene_name": "Palmitoyltransferase ZDHHC23",
  "term_label": "Golgi apparatus",
  "gene": "UniProtKB:Q8IYP9",
  "gene_symbol": "ZDHHC23"
}